{
  "gene_name": "Probable cysteine--tRNA ligase, mitochondrial",
  "term_label": "cytoplasm",
  "gene": "UniProtKB:Q9HA77",
  "term_id": "GO:0005737",
  "gene_symbol": "CARS2"
}